{
  "gene": "UniProtKB:O60359",
  "term_label": "AMPA glutamate receptor complex",
  "gene_symbol": "CACNG3",
  "gene_name": "Voltage-dependent calcium channel gamma-3 subunit",
  "term_id": "GO:0032281"
}